regulation of cytoplasmic pattern recognition receptor signaling pathway [GO:0039531] (BP) Also known as: regulation of cytosolic pattern recognition receptor signaling pathway, regulation of MAV signaling, regulation of viral-induced cytoplasmic pattern recognition receptor signaling pathway, regulation of viral-induced cytoplasmic pattern recognition receptor signalling pathway Sources: GOC:bf, GOC:jl Definition: Any process that modulates the frequency, rate or extent of a cytoplasmic pattern recognition receptor signaling pathway. Relationships: is_a regulation of pattern recognition receptor signaling pathway [GO:0062207]; is a type of regulation of intracellular signal transduction [GO:1902531]; regulates GO:0002753 Subtypes: regulation of toll-like receptor 3 signaling pathway [GO:0034139], GO:0034155, regulation of toll-like receptor 8 signaling pathway [GO:0034159], regulation of toll-like receptor 9 signaling pathway [GO:0034163], regulation of toll-like receptor 11 signaling pathway [GO:0034171], GO:0034175, regulation of toll-like receptor 13 signaling pathway [GO:0034179], negative regulation of cytoplasmic pattern recognition receptor signaling pathway [GO:0039532], GO:0039533, GO:0039535, regulation of nucleotide-binding domain, leucine rich repeat containing receptor signaling pathway [GO:0070424], regulation of inflammasome-mediated signaling pathway [GO:0141085], positive regulation of cGAS/STING signaling pathway [GO:0141111]